{
  "term_id": "GO:0098609",
  "gene": "UniProtKB:Q9BWV1",
  "term_label": "cell-cell adhesion",
  "gene_name": "Brother of CDO",
  "gene_symbol": "BOC"
}